{
  "gene": "UniProtKB:Q9UHG0",
  "term_label": "dendrite morphogenesis",
  "gene_symbol": "DCDC2",
  "gene_name": "Doublecortin domain-containing protein 2",
  "term_id": "GO:0048813"
}